{
  "term_id": "GO:0007286",
  "gene_name": "RIMS-binding protein 3C",
  "gene_symbol": "RIMBP3C",
  "term_label": "spermatid development",
  "gene": "UniProtKB:A6NJZ7"
}